{
  "term_label": "nucleus",
  "gene_name": "Dual specificity tyrosine-phosphorylation-regulated kinase 1A",
  "gene": "UniProtKB:Q13627",
  "gene_symbol": "DYRK1A",
  "term_id": "GO:0005634"
}